{
  "gene": "UniProtKB:Q9NVE7",
  "gene_symbol": "PANK4",
  "gene_name": "4'-phosphopantetheine phosphatase",
  "term_id": "GO:0005829",
  "term_label": "cytosol"
}